{
  "term_label": "adaptive immune response",
  "gene_name": "B-cell lymphoma_leukemia 10",
  "term_id": "GO:0002250",
  "gene_symbol": "BCL10",
  "gene": "UniProtKB:O95999"
}